regulation of glucuronoarabinoxylan catabolic process [GO:2000918] (biological process) Relationships: is a type of GO:2000915; is a type of regulation of arabinoxylan-containing compound catabolic process [GO:2000921]; regulates GO:2000887 Sources: GOC:mengo_curators Definition: Any process that modulates the frequency, rate or extent of glucuronoarabinoxylan catabolic process. Subtypes: negative regulation of glucuronoarabinoxylan catabolic process [GO:2000919], positive regulation of glucuronoarabinoxylan catabolic process [GO:2000920] Also known as: regulation of glucuronoarabinoxylan catabolism